{
  "term_id": "GO:0003688",
  "gene_symbol": "ORC5",
  "gene": "UniProtKB:O43913",
  "gene_name": "Origin recognition complex subunit 5",
  "term_label": "DNA replication origin binding"
}